{
  "term_id": "UNKNOWN:0002",
  "gene_name": "Brain and acute leukemia cytoplasmic protein",
  "gene_symbol": "BAALC",
  "gene": "UniProtKB:Q8WXS3",
  "term_label": "Unknown biological process"
}